BMP signaling pathway [GO:0030509] (biological process) Definition: The series of molecular signals initiated by the binding of a member of the BMP (bone morphogenetic protein) family to a receptor on the surface of a target cell, and ending with the regulation of a downstream cellular process, e.g. transcription. References: PMID:17428827 Sources: GOC:signaling, ISBN:0878932437 Regulation: regulated by GO:0030510; RO_0002213 by positive regulation of BMP signaling pathway [GO:0030513]; negatively regulated by GO:0030514 Also known as: BMP signalling pathway, bone morphogenetic protein signaling pathway, bone morphogenetic protein signalling pathway, decapentaplegic receptor signaling pathway, decapentaplegic receptor signalling pathway, decapentaplegic signaling pathway, dpp receptor signaling pathway, dpp receptor signalling pathway, dpp signaling pathway, BMP receptor signaling pathway Relationships: is a type of transforming growth factor beta receptor superfamily signaling pathway [GO:0141091]; is part of GO:0071773